negative regulation of I-kappaB phosphorylation [GO:1903720] (biological process) Definition: Any process that stops, prevents or reduces the frequency, rate or extent of I-kappaB phosphorylation. References: PMID:23675531 Sources: GOC:TermGenie, GO_REF:0000058 Also known as: negative regulation of IKB phosphorylation, negative regulation of IkappaB phosphorylation, negative regulation of inhibitor of NF-kappaB phosphorylation, negative regulation of inhibitor of kappaB phosphorylation, inhibition of I-kappaB phosphorylation, inhibition of IKB phosphorylation, inhibition of IkappaB phosphorylation, inhibition of inhibitor of NF-kappaB phosphorylation, inhibition of inhibitor of kappaB phosphorylation Relationships: is a type of negative regulation of protein phosphorylation [GO:0001933]; is a type of regulation of I-kappaB phosphorylation [GO:1903719]; negatively regulates I-kappaB phosphorylation [GO:0007252]